{
  "gene_name": "Probable mitochondrial glutathione transporter SLC25A40",
  "term_id": "GO:0005739",
  "gene": "UniProtKB:Q8TBP6",
  "term_label": "mitochondrion",
  "gene_symbol": "SLC25A40"
}